{
  "gene_name": "Double-stranded RNA-binding protein Staufen homolog 1",
  "gene": "UniProtKB:O95793",
  "term_label": "plasma membrane",
  "term_id": "GO:0005886",
  "gene_symbol": "STAU1"
}